{
  "gene_name": "Small ribosomal subunit protein uS13",
  "gene": "UniProtKB:P62269",
  "gene_symbol": "RPS18",
  "term_id": "GO:0005829",
  "term_label": "cytosol"
}